response to immobilization stress [GO:0035902] (biological process) Also known as: response to immobilisation stress, response to restraint stress Subtypes: cellular response to immobilization stress [GO:0035903], response to immobilization stress combined with electrical stimulus [GO:1990781], GO:1990785 Relationships: is a type of response to stress [GO:0006950] References: PMID:17683801, PMID:19893991 Sources: GOC:bf Definition: Any process that results in a change in state or activity of a cell or an organism (in terms of movement, secretion, enzyme production, gene expression, etc.) as a result of being rendered immobile.